{
  "gene_symbol": "NTF4",
  "term_label": "synaptic vesicle",
  "term_id": "GO:0008021",
  "gene": "UniProtKB:P34130",
  "gene_name": "Neurotrophin-4"
}